{
  "gene_symbol": "KRT6C",
  "term_id": "GO:0045109",
  "term_label": "intermediate filament organization",
  "gene_name": "Keratin, type II cytoskeletal 6C",
  "gene": "UniProtKB:P48668"
}